hemostasis [GO:0007599] (BP) Relationships: is a type of regulation of body fluid levels [GO:0050878] Subtypes: GO:0007596, GO:0042381 Definition: The stopping of bleeding (loss of body fluid) or the arrest of the circulation to an organ or part. Regulation: regulated by GO:1900046; negatively regulated by negative regulation of hemostasis [GO:1900047]; positively regulated by positive regulation of hemostasis [GO:1900048] Sources: ISBN:0198506732